mechanoreceptor differentiation involved in mechanosensory epithelium regeneration [GO:0070656] (biological process) Relationships: is a type of mechanoreceptor differentiation [GO:0042490]; is part of mechanosensory epithelium regeneration [GO:0070655] Definition: Differentiation of new mechanoreceptors to replace those lost or destroyed by injury. References: PMID:19381250 Sources: GOC:dsf Subtypes: neuromast hair cell differentiation involved in neuromast regeneration [GO:0070658], inner ear receptor cell differentiation involved in inner ear sensory epithelium regeneration [GO:0070660]